{
  "term_id": "GO:0015862",
  "term_label": "uridine transmembrane transport",
  "gene_name": "Equilibrative nucleoside transporter 2",
  "gene": "UniProtKB:Q14542",
  "gene_symbol": "SLC29A2"
}